protein deglycase activity [GO:0036524] (molecular function) Also known as: glyoxylase III, protein deglycating enzyme Definition: Catalysis of the removal of a sugar or dicarbonyl from a glycated L-arginine, L-lysine or L-cysteine residue within proteins that have been attacked and modified by glyoxal or 2-oxopropanal. References: PMID:14568004, PMID:25416785, PMID:26873906 Sources: EC:3.5.1.124, GOC:PARL, GOC:bf Relationships: is a type of hydrolase activity, acting on carbon-nitrogen (but not peptide) bonds, in linear amides [GO:0016811]; is a type of catalytic activity, acting on a protein [GO:0140096]